{
  "gene_symbol": "MRPS31",
  "gene_name": "Small ribosomal subunit protein mS31",
  "gene": "UniProtKB:Q92665",
  "term_id": "UNKNOWN:0001",
  "term_label": "Unknown molecular function"
}